{
  "gene_symbol": "LYZL2",
  "term_label": "Unknown cellular component",
  "gene_name": "Lysozyme-like protein 2",
  "term_id": "UNKNOWN:0003",
  "gene": "UniProtKB:Q7Z4W2"
}